{
  "gene_symbol": "MEIS2",
  "term_label": "positive regulation of cell population proliferation",
  "gene_name": "Homeobox protein Meis2",
  "term_id": "GO:0008284",
  "gene": "UniProtKB:O14770"
}